{
  "gene_symbol": "DGKK",
  "term_id": "GO:0004143",
  "gene": "UniProtKB:Q5KSL6",
  "term_label": "ATP-dependent diacylglycerol kinase activity",
  "gene_name": "Diacylglycerol kinase kappa"
}